{
  "term_label": "chromatin remodeling",
  "gene": "UniProtKB:Q96LA8",
  "gene_symbol": "PRMT6",
  "term_id": "GO:0006338",
  "gene_name": "Protein arginine N-methyltransferase 6"
}